{
  "gene": "UniProtKB:Q6ZNK6",
  "term_id": "GO:0035800",
  "gene_name": "TRAF-interacting protein with FHA domain-containing protein B",
  "gene_symbol": "TIFAB",
  "term_label": "deubiquitinase activator activity"
}